{
  "gene_symbol": "SLC48A1",
  "gene_name": "Heme transporter HRG1",
  "term_label": "plasma membrane",
  "term_id": "GO:0005886",
  "gene": "UniProtKB:Q6P1K1"
}